{
  "gene": "UniProtKB:P14151",
  "gene_name": "L-selectin",
  "gene_symbol": "SELL",
  "term_label": "response to cytokine",
  "term_id": "GO:0034097"
}